{
  "gene_name": "Transcription factor JunD",
  "term_id": "GO:0000981",
  "gene": "UniProtKB:P17535",
  "gene_symbol": "JUND",
  "term_label": "DNA-binding transcription factor activity, RNA polymerase II-specific"
}